(3R)-3-isopropenyl-6-oxoheptanoate:CoA ligase (ADP-forming) activity [GO:0052687] (MF) Also known as: 3-isopropenyl-6-oxoheptanoyl-CoA synthetase activity Definition: Catalysis of the reaction: (3R)-3-isopropenyl-6-oxoheptanoate + CoA-SH + ATP = H2O + ADP + phosphate + (3R)-3-isopropenyl-6-oxoheptanoyl-CoA. Sources: KEGG_REACTION:R06396 Relationships: is a type of CoA-ligase activity [GO:0016405]; is a type of GO:0016878